[protein]-asparagine 3-dioxygenase activity [GO:0036140] (molecular function) Definition: Catalysis of the reaction: peptidyl L-asparagine + 2-oxoglutarate + O2 = peptidyl 3-hydroxy-L-asparagine + succinate + CO2. Also known as: peptidyl-asparagine 3-dioxygenase activity, hypoxia-inducible factor-asparagine oxygenase activity References: PMID:12215170 Sources: GOC:reh, RHEA:54260 Relationships: is a type of 2-oxoglutarate-dependent dioxygenase activity [GO:0016706]; is a type of catalytic activity, acting on a protein [GO:0140096]